5-methyl-5,6,7,8-tetrahydromethanopterin-dependent methyltransferase activity [GO:0042086] (molecular function) Definition: Catalysis of the transfer of a methyl group to an acceptor molecule, dependent on the presence of 5-methyl-5,6,7,8-tetrahydromethanopterin. Sources: GOC:ai Relationships: is a type of methyltransferase activity [GO:0008168] Subtypes: tetrahydromethanopterin S-methyltransferase activity [GO:0030269]